{
  "gene_symbol": "ATG4C",
  "term_id": "GO:0019786",
  "gene_name": "Cysteine protease ATG4C",
  "term_label": "protein-phosphatidylethanolamide deconjugating activity",
  "gene": "UniProtKB:Q96DT6"
}